acetate ester transport [GO:1901374] (BP) Relationships: is a type of transport [GO:0006810] Sources: GOC:TermGenie Subtypes: acetylcholine transport [GO:0015870] Definition: The directed movement of an acetate ester into, out of or within a cell, or between cells, by means of some agent such as a transporter or pore.